ventricular septum morphogenesis [GO:0060412] (biological process) Also known as: interventricular septum morphogenesis Subtypes: ventricular septum intermedium morphogenesis [GO:0003288] Definition: The developmental process in which a ventricular septum is generated and organized. A ventricular septum is an anatomical structure that separates the lower chambers (ventricles) of the heart from one another. Relationships: is a type of cardiac septum morphogenesis [GO:0060411]; is part of ventricular septum development [GO:0003281] Sources: GOC:dph